{
  "gene_symbol": "PRL",
  "gene": "UniProtKB:P01236",
  "term_label": "female pregnancy",
  "gene_name": "Prolactin",
  "term_id": "GO:0007565"
}